{
  "gene_symbol": "PTPN23",
  "term_label": "endocytic recycling",
  "gene": "UniProtKB:Q9H3S7",
  "term_id": "GO:0032456",
  "gene_name": "Tyrosine-protein phosphatase non-receptor type 23"
}